hemozoin formation complex [GO:0160092] (cellular component) Relationships: is a type of protein-containing complex [GO:0032991] References: PMID:23471987 Definition: A protein-containing complex involved in hemoglobin degradation and detoxification of heme in the food vacuole during the asexual blood stage of a Plasmodium. It is composed of at least falcipains FP2A and/or FP2B, plasmepsins PMII, PMIII/HAP and PMIV, heme detoxifying protein HDP and falcilysin FLN.